{
  "gene_symbol": "ADAMTS13",
  "gene_name": "A disintegrin and metalloproteinase with thrombospondin motifs 13",
  "gene": "UniProtKB:Q76LX8",
  "term_id": "GO:0030198",
  "term_label": "extracellular matrix organization"
}